{
  "gene_name": "Guanine nucleotide-binding protein G(I)_G(S)_G(T) subunit beta-2",
  "term_id": "GO:0005834",
  "gene": "UniProtKB:P62879",
  "gene_symbol": "GNB2",
  "term_label": "heterotrimeric G-protein complex"
}